arsenite transport [GO:0015700] (biological process) Subtypes: arsenate ion transmembrane transport [GO:1901684] Definition: The directed movement of arsenite into, out of or within a cell, or between cells, by means of some agent such as a transporter or pore. Relationships: is a type of transport [GO:0006810] Sources: GOC:krc